T-helper 17 cell lineage commitment [GO:0072540] (biological process) Also known as: T-helper 17 cell fate commitment, Th17 cell lineage commitment, Th17 fate commitment Sources: CL:0000899, GOC:BHF, GOC:ebc Definition: The process in which a CD4-positive, alpha-beta T cell becomes committed to becoming a T-helper 17 cell, a CD4-positive, alpha-beta T cell with the phenotype RORgamma-t-positive that produces IL-17. Regulation: regulated by regulation of T-helper 17 cell lineage commitment [GO:2000328]; negatively regulated by GO:2000329; positively regulated by positive regulation of T-helper 17 cell lineage commitment [GO:2000330] Relationships: is a type of T-helper cell lineage commitment [GO:0002295]; is part of GO:0072539